mitochondrial electron transport, succinate to ubiquinone [GO:0006121] (biological process) Sources: ISBN:0716731363 Relationships: is a type of GO:0019646; BFO_0000050 mitochondrial ATP synthesis coupled electron transport [GO:0042775] Definition: The transfer of electrons from succinate to ubiquinone that occurs during oxidative phosphorylation, mediated by the multisubunit enzyme known as complex II. Also known as: mitochondrial electron transport, succinate to coenzyme Q, oxidative phosphorylation, succinate to ubiquinone, complex II (succinate to ubiquinone)